{
  "term_label": "Unknown molecular function",
  "gene": "UniProtKB:A0A0J9YXM7",
  "term_id": "UNKNOWN:0001",
  "gene_name": "T cell receptor beta joining 1-5",
  "gene_symbol": "TRBJ1-5"
}